{
  "term_id": "GO:0005925",
  "term_label": "focal adhesion",
  "gene_symbol": "LASP1",
  "gene_name": "LIM and SH3 domain protein 1",
  "gene": "UniProtKB:Q14847"
}